{
  "term_id": "GO:0022625",
  "gene_name": "Ribosomal protein uL16-like",
  "gene_symbol": "RPL10L",
  "term_label": "cytosolic large ribosomal subunit",
  "gene": "UniProtKB:Q96L21"
}